{
  "term_label": "sensory perception of smell",
  "gene_symbol": "OR5B2",
  "term_id": "GO:0007608",
  "gene_name": "Olfactory receptor 5B2",
  "gene": "UniProtKB:Q96R09"
}